neuromast development [GO:0048884] (biological process) Sources: ISBN:0125296509 Definition: The process whose specific outcome is the progression of the neuromast over time, from its formation to the mature structure. The neuromast is the sensory organ of the lateral line and is composed of a population of sensory hair cells, and nonsensory supporting cells and mantle cells. Neuromasts are located superficially on the epithelium or in lateral line canals. Relationships: is a type of GO:0007423; is part of GO:0048882 Subtypes: anterior lateral line neuromast development [GO:0048901], posterior lateral line neuromast development [GO:0048919]